{
  "gene_name": "Homeobox protein aristaless-like 3",
  "gene_symbol": "ALX3",
  "term_label": "nucleus",
  "gene": "UniProtKB:O95076",
  "term_id": "GO:0005634"
}